{
  "gene_name": "Calcium_calmodulin-dependent protein kinase type II subunit alpha",
  "term_label": "postsynaptic density",
  "gene": "UniProtKB:Q9UQM7",
  "gene_symbol": "CAMK2A",
  "term_id": "GO:0014069"
}